P granule [GO:0043186] (cellular component) Relationships: is a type of GO:0036464; BFO_0000050 GO:0060293 Also known as: germline granule, nuage, polar granule Subtypes: pi-body [GO:0071546], piP-body [GO:0071547] Definition: A small cytoplasmic, non-membranous RNA/protein complex aggregate in the primordial germ cells of many higher eukaryotes. References: PMID:11262230 Sources: GOC:dph, GOC:kmv